{
  "gene_name": "Ski-like protein",
  "term_label": "transcription regulator complex",
  "gene": "UniProtKB:P12757",
  "gene_symbol": "SKIL",
  "term_id": "GO:0005667"
}